cAMP deaminase activity [GO:0090612] (molecular function) References: PMID:24074367 Sources: RHEA:22908 Definition: Catalysis of the reaction: cyclic adenosine monophosphate + H2O = cyclic inosine monophosphate + NH3. Relationships: is a type of hydrolase activity, acting on carbon-nitrogen (but not peptide) bonds, in cyclic amidines [GO:0016814]; is a type of deaminase activity [GO:0019239] Also known as: cyclic adenosine monophosphate deaminase activity